lung connective tissue development [GO:0060427] (biological process) Relationships: is a type of connective tissue development [GO:0061448]; is part of lung development [GO:0030324] Also known as: pulmonary connective tissue development Definition: The biological process whose specific outcome is the progression of lung connective tissue from an initial condition to its mature state. This process begins with the formation of lung connective tissue and ends with the mature structure. The lung connective tissue is a material made up of fibers forming a framework and support structure for the lungs. Sources: GOC:dph, GOC:mtg_lung